{
  "gene_name": "Pancreatic polypeptide prohormone",
  "gene_symbol": "PPY",
  "gene": "UniProtKB:P01298",
  "term_id": "GO:0007218",
  "term_label": "neuropeptide signaling pathway"
}